cardiac right ventricle formation [GO:0003219] (biological process) Sources: GOC:mtg_heart Definition: The developmental process pertaining to the initial formation of a right cardiac ventricle from unspecified parts. Relationships: is a type of cardiac ventricle formation [GO:0003211]; BFO_0000050 cardiac right ventricle morphogenesis [GO:0003215]